multi-ciliated epithelial cell differentiation [GO:1903251] (biological process) Definition: The process in which a relatively unspecialized cell acquires the specialized features of a multi-ciliated epithelial cell. References: PMID:22231168, PMID:24934224 Sources: GOC:TermGenie, GOC:sp, GO_REF:0000086 Also known as: multiciliate cell differentiation Relationships: is a type of columnar/cuboidal epithelial cell differentiation [GO:0002065] Subtypes: lung ciliated cell differentiation [GO:0061141]